{
  "gene": "UniProtKB:O15235",
  "term_label": "translation",
  "gene_symbol": "MRPS12",
  "term_id": "GO:0006412",
  "gene_name": "Small ribosomal subunit protein uS12m"
}